{
  "gene_name": "Uncharacterized protein",
  "term_id": "UNKNOWN:0002",
  "gene": "UniProtKB:A0A669KAW2",
  "gene_symbol": "A0A669KAW2",
  "term_label": "Unknown biological process"
}